{
  "term_id": "UNKNOWN:0003",
  "gene": "UniProtKB:A9Z1Z3",
  "term_label": "Unknown cellular component",
  "gene_symbol": "FER1L4",
  "gene_name": "Fer-1-like protein 4"
}